{
  "gene_name": "Huntingtin-interacting protein M",
  "gene_symbol": "H2AP",
  "term_label": "structural constituent of chromatin",
  "gene": "UniProtKB:O75409",
  "term_id": "GO:0030527"
}